regulation of plasma membrane repair [GO:1905684] (biological process) Definition: Any process that modulates the frequency, rate or extent of plasma membrane repair. References: PMID:22940583 Sources: GOC:TermGenie, GOC:bhm, GO_REF:0000058 Relationships: is a type of GO:1903729; regulates plasma membrane repair [GO:0001778] Subtypes: negative regulation of plasma membrane repair [GO:1905685], positive regulation of plasma membrane repair [GO:1905686]